{
  "gene_name": "Insulin-like growth factor-binding protein 5",
  "term_label": "insulin-like growth factor I binding",
  "gene_symbol": "IGFBP5",
  "gene": "UniProtKB:P24593",
  "term_id": "GO:0031994"
}